{
  "gene_name": "Uncharacterized protein IDI2-AS1",
  "term_id": "UNKNOWN:0001",
  "gene": "UniProtKB:Q9NZ38",
  "term_label": "Unknown molecular function",
  "gene_symbol": "IDI2-AS1"
}